{
  "gene_name": "Cytochrome P450 1B1",
  "gene": "UniProtKB:Q16678",
  "gene_symbol": "CYP1B1",
  "term_label": "steroid hydroxylase activity",
  "term_id": "GO:0008395"
}